{
  "term_id": "GO:0005856",
  "gene": "UniProtKB:Q15323",
  "term_label": "cytoskeleton",
  "gene_symbol": "KRT31",
  "gene_name": "Keratin, type I cuticular Ha1"
}